exomer complex [GO:0034044] (CC) References: PMID:16498409, PMID:17000877 Definition: A protein complex that forms a coat structure on vesicles involved in exocytosis of proteins from the trans-Golgi network to the cell surface; in Saccharomyces, the complex contains Chs5p, Chs6p, and Chs6p paralogues. Relationships: is a type of protein-containing complex [GO:0032991]; is part of Golgi apparatus [GO:0005794]; BFO_0000050 GO:0030140